male germ cell proliferation [GO:0002176] (biological process) Relationships: is a type of germ cell proliferation [GO:0036093] Regulation: regulated by regulation of male germ cell proliferation [GO:2000254]; negatively regulated by negative regulation of male germ cell proliferation [GO:2000255]; positively regulated by positive regulation of male germ cell proliferation [GO:2000256] Sources: GOC:hjd Definition: The multiplication or reproduction of male germ cells, resulting in the expansion of a cell population.